{
  "gene_symbol": "GUCA2B",
  "gene": "UniProtKB:Q16661",
  "gene_name": "Guanylate cyclase activator 2B",
  "term_label": "Unknown cellular component",
  "term_id": "UNKNOWN:0003"
}